tRNA wobble base modification [GO:0002097] (biological process) References: PMID:28812932 Relationships: is a type of GO:0006400 Subtypes: GO:0002098, tRNA wobble guanine modification [GO:0002099], tRNA wobble adenosine to inosine editing [GO:0002100], tRNA wobble cytosine modification [GO:0002101] Definition: The process in which the nucleotide at position 34 in the anticodon of a tRNA is post-transcriptionally modified. The wobble nucleoside of the tRNA sequence  (position 34) corresponds to the first position of the anticodon.